{
  "gene": "UniProtKB:Q01118",
  "gene_symbol": "SCN7A",
  "term_id": "GO:0086002",
  "gene_name": "Sodium channel protein type 7 subunit alpha",
  "term_label": "cardiac muscle cell action potential involved in contraction"
}